coumarin biosynthetic process [GO:0009805] (biological process) Subtypes: esculetin biosynthetic process [GO:0033493], GO:0043642, sideretin biosynthesis [GO:0106146], GO:0106147, 4-hydroxycoumarin biosynthetic process [GO:1901884] Also known as: coumarin anabolism, coumarin biosynthesis, coumarin formation, coumarin synthesis Relationships: is a type of phenylpropanoid biosynthetic process [GO:0009699]; is a type of coumarin metabolic process [GO:0009804] Definition: The chemical reactions and pathways resulting in the formation of coumarins, a class of compounds derived from the phenylacrylic skeleton of cinnamic acids. Sources: GOC:lr, GOC:yl